{
  "gene": "UniProtKB:Q9BT88",
  "gene_symbol": "SYT11",
  "term_label": "calcium ion sensor activity",
  "gene_name": "Synaptotagmin-11",
  "term_id": "GO:0061891"
}